{
  "gene_name": "Zinc finger protein 230",
  "term_label": "Unknown biological process",
  "term_id": "UNKNOWN:0002",
  "gene_symbol": "ZNF230",
  "gene": "UniProtKB:Q9UIE0"
}